{
  "gene_symbol": "NOL11",
  "gene_name": "Nucleolar protein 11",
  "term_label": "maturation of SSU-rRNA",
  "term_id": "GO:0030490",
  "gene": "UniProtKB:Q9H8H0"
}